{
  "gene_symbol": "TNFSF14",
  "term_id": "GO:0043123",
  "gene": "UniProtKB:O43557",
  "term_label": "positive regulation of canonical NF-kappaB signal transduction",
  "gene_name": "Tumor necrosis factor ligand superfamily member 14"
}